{
  "gene": "UniProtKB:Q8NGL2",
  "gene_name": "Olfactory receptor 5L1",
  "gene_symbol": "OR5L1",
  "term_id": "GO:0007608",
  "term_label": "sensory perception of smell"
}